{
  "term_label": "rescue of stalled ribosome",
  "gene_symbol": "RNF25",
  "gene_name": "E3 ubiquitin-protein ligase RNF25",
  "gene": "UniProtKB:Q96BH1",
  "term_id": "GO:0072344"
}